{
  "gene_name": "Exportin-4",
  "term_id": "GO:0005049",
  "term_label": "nuclear export signal receptor activity",
  "gene_symbol": "XPO4",
  "gene": "UniProtKB:Q9C0E2"
}